galactosylgalactosylxylosylprotein 3-beta-glucuronosyltransferase activity [GO:0015018] (molecular function) Relationships: is a type of GO:0015020 Definition: Catalysis of the reaction: 3-O-(beta-D-galactosyl-(1->3)-beta-D-galactosyl-(1->4)-beta-D-xylosyl)-L-seryl-[protein] + UDP-alpha-D-glucuronate = 3-O-(beta-D-GlcA-(1->3)-beta-D-Gal-(1->3)-beta-D-Gal-(1->4)-beta-D-Xyl)-L-seryl-[protein] + H+ + UDP. Sources: EC:2.4.1.135 Also known as: glucuronosyltransferase I activity, UDP-glucuronate:3-beta-D-galactosyl-4-beta-D-galactosyl-O-beta-D-xylosyl-protein D-glucuronosyltransferase activity, UDPglucuronate:3-beta-D-galactosyl-4-beta-D-galactosyl-O-beta-D-xylosyl-protein D-glucuronosyltransferase activity, uridine diphosphate glucuronic acid:acceptor glucuronosyltransferase activity